{
  "term_id": "GO:0016605",
  "gene_symbol": "N4BP1",
  "gene_name": "NEDD4-binding protein 1",
  "term_label": "PML body",
  "gene": "UniProtKB:O75113"
}